{
  "gene_symbol": "TYMS",
  "term_label": "thymidylate synthase activity",
  "term_id": "GO:0004799",
  "gene": "UniProtKB:P04818",
  "gene_name": "Thymidylate synthase"
}